{
  "gene": "UniProtKB:P35542",
  "gene_name": "Serum amyloid A-4 protein",
  "term_id": "UNKNOWN:0002",
  "gene_symbol": "SAA4",
  "term_label": "Unknown biological process"
}